{
  "gene_symbol": "PRAMEF14",
  "term_id": "GO:0043161",
  "gene": "UniProtKB:Q5SWL7",
  "term_label": "proteasome-mediated ubiquitin-dependent protein catabolic process",
  "gene_name": "PRAME family member 14"
}